regulation of cytoplasmic translational elongation through polyproline stretches [GO:1903270] (biological process) Subtypes: negative regulation of cytoplasmic translational elongation through polyproline stretches [GO:1903271], GO:1903272 Definition: Any process that modulates the frequency, rate or extent of cytoplasmic translational elongation through polyproline stretches. Relationships: is a type of regulation of cytoplasmic translational elongation [GO:1900247]; regulates cytoplasmic translational elongation through polyproline stretches [GO:0097622] References: PMID:24923804 Sources: GOC:TermGenie, GO_REF:0000058